{
  "term_id": "GO:0016020",
  "term_label": "membrane",
  "gene": "UniProtKB:Q9H3M0",
  "gene_name": "Potassium voltage-gated channel subfamily F member 1",
  "gene_symbol": "KCNF1"
}